{
  "term_id": "GO:0005509",
  "gene": "UniProtKB:P33764",
  "term_label": "calcium ion binding",
  "gene_symbol": "S100A3",
  "gene_name": "Protein S100-A3"
}